{
  "gene_name": "Proton-coupled zinc antiporter SLC30A2",
  "term_label": "response to zinc ion",
  "gene_symbol": "SLC30A2",
  "gene": "UniProtKB:Q9BRI3",
  "term_id": "GO:0010043"
}